{
  "gene_name": "Twinfilin-1",
  "gene": "UniProtKB:Q12792",
  "term_id": "GO:0051015",
  "gene_symbol": "TWF1",
  "term_label": "actin filament binding"
}